{
  "term_id": "UNKNOWN:0003",
  "gene": "UniProtKB:Q7LFX5",
  "gene_name": "Carbohydrate sulfotransferase 15",
  "term_label": "Unknown cellular component",
  "gene_symbol": "CHST15"
}